{
  "gene_name": "Kv channel-interacting protein 4",
  "gene": "UniProtKB:Q6PIL6",
  "term_label": "potassium channel regulator activity",
  "term_id": "GO:0015459",
  "gene_symbol": "KCNIP4"
}